{
  "gene": "UniProtKB:P34969",
  "gene_name": "5-hydroxytryptamine receptor 7",
  "term_label": "plasma membrane",
  "term_id": "GO:0005886",
  "gene_symbol": "HTR7"
}